Mre11 complex assembly [GO:0072685] (biological process) Relationships: is a type of protein-containing complex assembly [GO:0065003] Also known as: MRN complex assembly, MRX complex assembly, RAD50-MRE11-NBN complex assembly, RMX complex assembly, Rad50 complex assembly, Rad50-Rad32-Nbs1 complex assembly References: PMID:19211838 Sources: GOC:mah Definition: The aggregation, arrangement and bonding together of a set of components to form an Mre11 complex, a trimeric protein complex that possesses endonuclease activity and is involved in meiotic recombination, DNA repair and checkpoint signaling.